{
  "term_id": "GO:0005523",
  "gene_name": "Tropomodulin-3",
  "gene": "UniProtKB:Q9NYL9",
  "term_label": "tropomyosin binding",
  "gene_symbol": "TMOD3"
}